RSC-type complex [GO:0016586] (cellular component) References: PMID:11937489, PMID:12672490, PMID:15870268, PMID:19355820, PMID:8980231 Sources: GOC:bhm Definition: A SWI/SNF-type complex that contains a bromodomain containing-protein, such as yeast Rsc1 or Rsc4 or mammalian PB1/BAF180. The RSC complex is generally recruited to RNA polymerase III promoters and is specifically recruited to RNA polymerase II promoters by transcriptional activators and repressors; it is also involved in non-homologous end joining. Relationships: is a type of SWI/SNF superfamily-type complex [GO:0070603] Also known as: PBAF complex, Polybromo- and BAF containing complex, SWI/SNF complex B